{
  "term_id": "GO:0007212",
  "gene_symbol": "DORIP1",
  "gene_name": "Uncharacterized protein C14orf28",
  "term_label": "G protein-coupled dopamine receptor signaling pathway",
  "gene": "UniProtKB:Q4W4Y0"
}